negative regulation of type I interferon-mediated signaling pathway [GO:0060339] (biological process) Also known as: negative regulation of type I interferon-mediated signalling pathway Sources: GOC:dph Definition: Any process that decreases the rate, frequency or extent of a type I interferon-mediated signaling pathway. Relationships: is a type of GO:0001960; is a type of GO:0045824; is a type of regulation of type I interferon-mediated signaling pathway [GO:0060338]; negatively regulates type I interferon-mediated signaling pathway [GO:0060337]